distal stomach smooth muscle contraction [GO:0014828] (biological process) Definition: A process in which force is generated within smooth muscle tissue, resulting in a change in muscle geometry. This process occurs in the distal stomach. Force generation involves a chemo-mechanical energy conversion step that is carried out by the actin/myosin complex activity, which generates force through ATP hydrolysis. The distal stomach is composed of the lower body and antrum and develops strong peristaltic phasic contractions that increase in amplitude as they propagate toward the pylorus. References: PMID:30252381 Sources: GOC:mtg_muscle Relationships: is a type of phasic smooth muscle contraction [GO:0014821]; is a type of stomach smooth muscle contraction [GO:0120063] Subtypes: GO:0014845, GO:0120064